{
  "term_id": "GO:0005634",
  "gene_name": "Parathymosin",
  "gene": "UniProtKB:P20962",
  "gene_symbol": "PTMS",
  "term_label": "nucleus"
}